{
  "term_id": "UNKNOWN:0003",
  "gene": "UniProtKB:Q52M75",
  "term_label": "Unknown cellular component",
  "gene_symbol": "LINC01554",
  "gene_name": "Putative uncharacterized protein encoded by LINC01554"
}